negative regulation of non-professional antigen presenting cell antigen processing and presentation [GO:0002620] (biological process) Relationships: is a type of GO:0002578; is a type of GO:0002619; negatively regulates non-professional antigen presenting cell antigen processing and presentation [GO:0002473] Also known as: down regulation of non-professional antigen presenting cell antigen processing and presentation, down-regulation of non-professional antigen presenting cell antigen processing and presentation, downregulation of non-professional antigen presenting cell antigen processing and presentation, inhibition of non-professional antigen presenting cell antigen processing and presentation Definition: Any process that stops, prevents, or reduces the frequency, rate, or extent of non-professional antigen presenting cell antigen processing and presentation. Sources: GOC:add